{
  "gene": "UniProtKB:Q9H6L4",
  "gene_name": "Armadillo repeat-containing protein 7",
  "term_label": "Unknown cellular component",
  "term_id": "UNKNOWN:0003",
  "gene_symbol": "ARMC7"
}